{
  "term_label": "cell migration",
  "gene": "UniProtKB:P18827",
  "term_id": "GO:0016477",
  "gene_name": "Syndecan-1",
  "gene_symbol": "SDC1"
}